abscisic aldehyde oxidase activity [GO:0010293] (molecular function) Relationships: is a type of aryl-aldehyde oxidase activity [GO:0018488] Sources: RHEA:20529 Definition: Catalysis of the reaction: a 2-cis-(+)-abscisic aldehyde + H2O + O2 = 2-cis-(+)-abscisate + H+ + H2O2. Also known as: AAO3, AOdelta, abscisic-aldehyde oxidase activity, abscisic-aldehyde:oxygen oxidoreductase activity